{
  "gene": "UniProtKB:Q9Y584",
  "gene_name": "Mitochondrial import inner membrane translocase subunit Tim22",
  "term_id": "GO:0045039",
  "term_label": "protein insertion into mitochondrial inner membrane",
  "gene_symbol": "TIMM22"
}